{
  "gene": "UniProtKB:Q9H4M3",
  "gene_name": "F-box only protein 44",
  "term_label": "ubiquitin protein ligase activity",
  "gene_symbol": "FBXO44",
  "term_id": "GO:0061630"
}